{
  "gene_symbol": "ATG4A",
  "gene": "UniProtKB:Q8WYN0",
  "gene_name": "Cysteine protease ATG4A",
  "term_label": "protein-phosphatidylethanolamide deconjugating activity",
  "term_id": "GO:0019786"
}